{
  "gene_name": "Oligophrenin-1",
  "term_id": "GO:0051966",
  "gene_symbol": "OPHN1",
  "gene": "UniProtKB:O60890",
  "term_label": "regulation of synaptic transmission, glutamatergic"
}